{
  "term_label": "Unknown cellular component",
  "gene": "UniProtKB:Q9HCI6",
  "gene_name": "E3 SUMO-protein ligase KIAA1586",
  "gene_symbol": "KIAA1586",
  "term_id": "UNKNOWN:0003"
}